{
  "gene_symbol": "CEP170B",
  "term_id": "UNKNOWN:0001",
  "term_label": "Unknown molecular function",
  "gene": "UniProtKB:Q9Y4F5",
  "gene_name": "Centrosomal protein of 170 kDa protein B"
}